{
  "gene_name": "Arf-GAP with GTPase, ANK repeat and PH domain-containing protein 2",
  "gene": "UniProtKB:Q99490",
  "gene_symbol": "AGAP2",
  "term_id": "GO:0005737",
  "term_label": "cytoplasm"
}